{
  "gene": "UniProtKB:A0A075B713",
  "gene_name": "T cell receptor alpha joining 1 (non-functional) (Fragment)",
  "term_label": "Unknown biological process",
  "term_id": "UNKNOWN:0002",
  "gene_symbol": "TRAJ1"
}